intrinsic apoptotic signaling pathway in response to endoplasmic reticulum stress [GO:0070059] (biological process) Regulation: RO_0002211 by regulation of endoplasmic reticulum stress-induced intrinsic apoptotic signaling pathway [GO:1902235]; negatively regulated by GO:1902236; positively regulated by GO:1902237 Also known as: apoptosis in response to endoplasmic reticulum stress, ER stress-induced apoptosis, apoptosis in response to ER stress, apoptosis triggered by ER stress, endoplasmic reticulum stress-induced apoptosis, intrinsic apoptotic signaling pathway induced by endoplasmic reticulum stress Subtypes: neuron intrinsic apoptotic signaling pathway in response to endoplasmic reticulum stress [GO:0036483] Definition: The series of molecular signals in which an intracellular signal is conveyed to trigger the apoptotic death of a cell. The pathway is induced in response to a stimulus indicating endoplasmic reticulum (ER) stress, and ends when the execution phase of apoptosis is triggered. ER stress usually results from the accumulation of unfolded or misfolded proteins in the ER lumen. Relationships: is a type of GO:0034976; is a type of intrinsic apoptotic signaling pathway [GO:0097193] References: PMID:18701708 Sources: GOC:mah, GOC:mtg_apoptosis